defense response to tumor cell [GO:0002357] (biological process) Relationships: is a type of GO:0002347; is a type of defense response [GO:0006952] Definition: Reactions triggered in response to the presence of a tumor cell that act to protect the cell or organism. References: PMID:16730260 Sources: GOC:add, ISBN:0781735149